{
  "term_id": "GO:0000978",
  "term_label": "RNA polymerase II cis-regulatory region sequence-specific DNA binding",
  "gene_name": "POU domain, class 3, transcription factor 2",
  "gene": "UniProtKB:P20265",
  "gene_symbol": "POU3F2"
}